{
  "gene_name": "BolA-like protein 2",
  "gene_symbol": "BOLA2",
  "term_label": "intracellular iron ion homeostasis",
  "gene": "UniProtKB:Q9H3K6",
  "term_id": "GO:0006879"
}